positive regulation of translational initiation in response to osmotic stress [GO:0032064] (biological process) Definition: Any process that activates or increases the frequency, rate or extent of translation initiation, as a result of a stimulus indicating an increase or decrease in the concentration of solutes outside the organism or cell. Also known as: up regulation of translation initiation in response to osmotic stress, up-regulation of translation initiation in response to osmotic stress, upregulation of translation initiation in response to osmotic stress, activation of translation initiation in response to osmotic stress, stimulation of translation initiation in response to osmotic stress Sources: GOC:mah Relationships: is a type of positive regulation of translational initiation in response to stress [GO:0032058]; is a type of positive regulation of translation in response to osmotic stress [GO:0032062]; is a type of GO:0043561